{
  "term_id": "GO:0016020",
  "gene": "UniProtKB:P98073",
  "gene_symbol": "TMPRSS15",
  "term_label": "membrane",
  "gene_name": "Enteropeptidase"
}